{
  "term_id": "GO:0004308",
  "gene_name": "Sialidase-3",
  "gene_symbol": "NEU3",
  "term_label": "exo-alpha-sialidase activity",
  "gene": "UniProtKB:Q9UQ49"
}